{
  "gene": "UniProtKB:Q5I0G3",
  "term_id": "GO:0006107",
  "gene_name": "Putative malate dehydrogenase 1B",
  "gene_symbol": "MDH1B",
  "term_label": "oxaloacetate metabolic process"
}